{
  "gene_name": "AP-2 complex subunit beta",
  "term_id": "UNKNOWN:0003",
  "gene_symbol": "AP2B1",
  "term_label": "Unknown cellular component",
  "gene": "UniProtKB:P63010"
}